{
  "gene_name": "Testis-specific protein TEX28",
  "term_label": "Unknown molecular function",
  "term_id": "UNKNOWN:0001",
  "gene": "UniProtKB:O15482",
  "gene_symbol": "TEX28"
}